{
  "gene_name": "Aldo-keto reductase family 1 member B10",
  "term_label": "Unknown biological process",
  "term_id": "UNKNOWN:0002",
  "gene_symbol": "AKR1B10",
  "gene": "UniProtKB:O60218"
}